binding [GO:0005488] (molecular function) Definition: The selective, non-covalent, often stoichiometric, interaction of a molecule with one or more specific sites on another molecule. Regulation: regulated by regulation of binding [GO:0051098]; positively regulated by GO:0051099; negatively regulated by negative regulation of binding [GO:0051100] Subtypes: GO:0003676, chromatin binding [GO:0003682], antigen binding [GO:0003823], protein binding [GO:0005515], macrolide binding [GO:0005527], odorant binding [GO:0005549], lipid binding [GO:0008289], toxic substance binding [GO:0015643], amino acid binding [GO:0016597], intermediate filament binding [GO:0019215], carbohydrate binding [GO:0030246], pigment binding [GO:0031409], amide binding [GO:0033218], tetrahydrobiopterin binding [GO:0034617], GO:0035274, GO:0035275, GO:0036094, GO:0042277, hormone binding [GO:0042562], GO:0043176, kinetochore binding [GO:0043515], molybdopterin cofactor binding [GO:0043546], GO:0044877, host cell surface binding [GO:0046812], tetrapyrrole binding [GO:0046906], GO:0050809, extracellular matrix binding [GO:0050840], prosthetic group binding [GO:0051192], GO:0072341, polychlorinated biphenyl binding [GO:0097160], flavonoid binding [GO:0097243], GO:0097367, nucleoside phosphate binding [GO:1901265], catecholamine binding [GO:1901338], sulfur compound binding [GO:1901681], hydroquinone binding [GO:1902314], synthetic cannabinoid binding [GO:1904483], GO:1905594, GO:1990300 Sources: GOC:ceb, GOC:mah, ISBN:0198506732 Relationships: is a type of molecular_function [GO:0003674] Also known as: ligand